XPC complex [GO:0071942] (CC) Relationships: is a type of nucleotide-excision repair complex [GO:0000109] References: PMID:11279143, PMID:15964821, PMID:19941824 Definition: A nucleotide-excision repair complex that is involved in damage sensing during global genome nucleotide excision repair (GG-NER). It is part of the pre-incision (or initial recognition) complex bound to sites of DNA damage. In human, it is composed of XPC, RAD23B and CETN2.